{
  "gene_name": "Uncharacterized protein C10orf67, mitochondrial",
  "term_label": "Unknown molecular function",
  "gene_symbol": "C10orf67",
  "term_id": "UNKNOWN:0001",
  "gene": "UniProtKB:Q8IYJ2"
}